BH1 domain binding [GO:0051432] (molecular function) Definition: Binding to a BH1 protein domain, present in Bcl-2 family members. Proteins that act as inhibitors of apoptosis harbour at least three BH domains: BH1, BH2 and BH3; the BH1 and BH2 domains are found in all death antagonists of the Bcl-2 family but only in one class of death agonists. References: PMID:11048732, PMID:12133724, PMID:9020082, PMID:9704409 Sources: Prosite:PS01080 Relationships: is_a BH domain binding [GO:0051400]